{
  "gene_name": "Epididymal secretory protein E3-beta",
  "gene": "UniProtKB:P56851",
  "term_label": "Unknown biological process",
  "gene_symbol": "EDDM3B",
  "term_id": "UNKNOWN:0002"
}